transferase complex [GO:1990234] (cellular component) Subtypes: 1,3-beta-D-glucan synthase complex [GO:0000148], ubiquitin ligase complex [GO:0000151], EKC/KEOPS complex [GO:0000408], GO:0000506, palmitoyltransferase complex [GO:0002178], fatty-acyl-CoA synthase complex [GO:0005836], alpha,alpha-trehalose-phosphate synthase complex (UDP-forming) [GO:0005946], acetolactate synthase complex [GO:0005948], CAAX-protein geranylgeranyltransferase complex [GO:0005953], glycine cleavage complex [GO:0005960], protein farnesyltransferase complex [GO:0005965], Rab-protein geranylgeranyltransferase complex [GO:0005968], serine-pyruvate aminotransferase complex [GO:0005969], GO:0008250, acetate CoA-transferase complex [GO:0009329], cysteine synthase complex [GO:0009333], aspartate carbamoyltransferase complex [GO:0009347], riboflavin synthase complex [GO:0009349], imidazoleglycerol-phosphate synthase complex [GO:0009382], GO:0009923, GO:0010330, protein N-acetylglucosaminyltransferase complex [GO:0017122], ubiquitin conjugating enzyme complex [GO:0031371], mannosyltransferase complex [GO:0031501], 4-aminobutyrate transaminase complex [GO:0032144], GO:0032476, Atg12-Atg5-Atg16 complex [GO:0034274], methyltransferase complex [GO:0034708], fatty acid beta-oxidation multienzyme complex [GO:0036125], GO:0042765, methyl coenzyme M reductase complex [GO:0044674], oxoglutarate dehydrogenase complex [GO:0045252], methionine adenosyltransferase complex [GO:0048269], transferase complex, transferring phosphorus-containing groups [GO:0061695], inositol phosphoceramide synthase complex [GO:0070916], SUMO ligase complex [GO:0106068], EXT1-EXT2 complex [GO:0120504], tRNA-guanine transglycosylase complex [GO:0120507], 2-(3-amino-3-carboxypropyl)histidine synthase complex [GO:0120513], ATP-dependent citrate lyase complex [GO:0140615], GO:0160157, GO:0170069, GO:1902493, GO:1990228, iron-sulfur cluster transfer complex [GO:1990230], Bre1-Rad6 ubiquitin ligase complex [GO:1990302], UBR1-RAD6 ubiquitin ligase complex [GO:1990303], MUB1-RAD6-UBR2 ubiquitin ligase complex [GO:1990304], RAD6-UBR2 ubiquitin ligase complex [GO:1990305], RSP5-BUL ubiquitin ligase complex [GO:1990306], transnitrosylase complex [GO:1990658], GO:7770010 Definition: A protein complex capable of catalyzing the transfer of a group, e.g. a methyl group, glycosyl group, acyl group, phosphorus-containing, or other groups, from one compound (generally regarded as the donor) to another compound (generally regarded as the acceptor). Relationships: is a type of GO:1902494 References: PMID:16540464 Sources: GOC:bhm